acyl-CoA binding [GO:0120227] (molecular function) Relationships: is a type of GO:0033218; is a type of anion binding [GO:0043168]; is a type of nucleoside phosphate binding [GO:1901265]; is a type of heterocyclic compound binding [GO:1901363]; is_a GO:1901681 Subtypes: fatty-acyl-CoA binding [GO:0000062], succinyl-CoA binding [GO:0120226], GO:1905502 Sources: GOC:krc Definition: Binding to an acyl-CoA, a thioester that results from the formal condensation of the thiol group of coenzyme A with the carboxy group of any carboxylic acid. Also known as: acyl binding, acyl-coenzyme A binding